{
  "term_label": "regulation of DNA-templated transcription",
  "term_id": "GO:0006355",
  "gene_symbol": "KMT2E",
  "gene": "UniProtKB:Q8IZD2",
  "gene_name": "Inactive histone-lysine N-methyltransferase 2E"
}